{
  "gene_symbol": "MT1E",
  "term_label": "cellular response to copper ion",
  "term_id": "GO:0071280",
  "gene": "UniProtKB:P04732",
  "gene_name": "Metallothionein-1E"
}